negative regulation of multicellular organism growth [GO:0040015] (biological process) Relationships: is a type of regulation of multicellular organism growth [GO:0040014]; is a type of negative regulation of developmental growth [GO:0048640]; is a type of negative regulation of multicellular organismal process [GO:0051241]; RO_0002212 multicellular organism growth [GO:0035264] Sources: GOC:dph, GOC:ems, GOC:tb Also known as: negative regulation of body growth, negative regulation of body size Definition: Any process that stops, prevents, or reduces the frequency, rate or extent of growth of an organism to reach its usual body size.